{
  "term_label": "neuron migration",
  "term_id": "GO:0001764",
  "gene_symbol": "DISC1",
  "gene": "UniProtKB:Q9NRI5",
  "gene_name": "Disrupted in schizophrenia 1 protein"
}